{
  "gene": "UniProtKB:O14519",
  "term_label": "cytoplasm",
  "term_id": "GO:0005737",
  "gene_symbol": "CDK2AP1",
  "gene_name": "Cyclin-dependent kinase 2-associated protein 1"
}